{
  "gene_name": "Integrin-linked protein kinase",
  "term_id": "GO:0030154",
  "term_label": "cell differentiation",
  "gene_symbol": "ILK",
  "gene": "UniProtKB:Q13418"
}